{
  "gene_name": "60 kDa heat shock protein, mitochondrial",
  "gene_symbol": "HSPD1",
  "term_id": "GO:0051087",
  "term_label": "protein-folding chaperone binding",
  "gene": "UniProtKB:P10809"
}